assembly of large subunit precursor of preribosome [GO:1902626] (biological process) Definition: The aggregation, arrangement and bonding together of a set of components to form the large subunit precursor of the preribosome. Also known as: preribosome, large subunit precursor formation, 66S preribosome assembly, 66S preribosome formation Relationships: is a type of protein-RNA complex assembly [GO:0022618]; is part of ribosomal large subunit assembly [GO:0000027] Regulation: regulated by regulation of assembly of large subunit precursor of preribosome [GO:1902627]; positively regulated by positive regulation of assembly of large subunit precursor of preribosome [GO:1902628] References: PMID:22735702 Sources: GOC:TermGenie, GOC:di, GO_REF:0000079